{
  "gene": "UniProtKB:P10321",
  "term_label": "external side of plasma membrane",
  "gene_name": "HLA class I histocompatibility antigen, C alpha chain",
  "gene_symbol": "HLA-C",
  "term_id": "GO:0009897"
}